{
  "gene_name": "ATP-binding cassette sub-family D member 1",
  "gene_symbol": "ABCD1",
  "term_id": "GO:0007031",
  "term_label": "peroxisome organization",
  "gene": "UniProtKB:P33897"
}